face development [GO:0060324] (biological process) Definition: The biological process whose specific outcome is the progression of a face from an initial condition to its mature state. The face is the ventral division of the head. Sources: GOC:dph Relationships: is a type of anatomical structure development [GO:0048856]; is part of head development [GO:0060322]